{
  "term_id": "UNKNOWN:0003",
  "term_label": "Unknown cellular component",
  "gene_symbol": "AP3S2",
  "gene_name": "AP-3 complex subunit sigma-2",
  "gene": "UniProtKB:P59780"
}